{
  "gene_symbol": "MTHFD2",
  "gene": "UniProtKB:P13995",
  "term_id": "GO:0004487",
  "term_label": "methylenetetrahydrofolate dehydrogenase (NAD+) activity",
  "gene_name": "Bifunctional methylenetetrahydrofolate dehydrogenase_cyclohydrolase, mitochondrial"
}